{
  "term_label": "cytoplasm",
  "gene": "UniProtKB:Q9NQ48",
  "gene_name": "Leucine zipper transcription factor-like protein 1",
  "gene_symbol": "LZTFL1",
  "term_id": "GO:0005737"
}